{
  "gene_symbol": "KRTAP5-2",
  "gene_name": "Keratin-associated protein 5-2",
  "gene": "UniProtKB:Q701N4",
  "term_label": "Unknown cellular component",
  "term_id": "UNKNOWN:0003"
}